{
  "gene_symbol": "SYVN1",
  "gene": "UniProtKB:Q86TM6",
  "gene_name": "E3 ubiquitin-protein ligase synoviolin",
  "term_id": "GO:0043161",
  "term_label": "proteasome-mediated ubiquitin-dependent protein catabolic process"
}